{
  "gene_symbol": "CPEB2",
  "term_label": "mRNA regulatory element binding translation repressor activity",
  "term_id": "GO:0000900",
  "gene": "UniProtKB:Q7Z5Q1",
  "gene_name": "Cytoplasmic polyadenylation element-binding protein 2"
}